{
  "gene": "UniProtKB:Q96RT1",
  "gene_symbol": "ERBIN",
  "term_label": "negative regulation of nucleotide-binding oligomerization domain containing 2 signaling pathway",
  "term_id": "GO:0070433",
  "gene_name": "Erbin"
}